{
  "term_id": "GO:0005615",
  "gene_symbol": "ENPP2",
  "gene": "UniProtKB:Q13822",
  "term_label": "extracellular space",
  "gene_name": "Ectonucleotide pyrophosphatase_phosphodiesterase family member 2"
}